{
  "term_label": "hormone activity",
  "gene": "UniProtKB:A6NKQ9",
  "term_id": "GO:0005179",
  "gene_name": "Choriogonadotropin subunit beta variant 1",
  "gene_symbol": "CGB1"
}